carbon-oxygen lyase activity [GO:0016835] (molecular function) Relationships: is a type of lyase activity [GO:0016829] Also known as: other carbon-oxygen lyase activity Sources: EC:4.2.-.- Definition: Catalysis of the breakage of a carbon-oxygen bond. Subtypes: hydro-lyase activity [GO:0016836], carbon-oxygen lyase activity, acting on polysaccharides [GO:0016837], carbon-oxygen lyase activity, acting on phosphates [GO:0016838], isochorismate pyruvate lyase activity [GO:0043904], versicolorin B synthase activity [GO:0046572], carboxymethyloxysuccinate lyase activity [GO:0047772], O-acetylhomoserine sulfhydrylase activity [GO:0051009], 5'-deoxyribose-5-phosphate lyase activity [GO:0051575], GO:0070205, class I DNA-(apurinic or apyrimidinic site) endonuclease activity [GO:0140078]